{
  "term_label": "plasma membrane",
  "gene_symbol": "RND3",
  "gene": "UniProtKB:P61587",
  "gene_name": "Rho-related GTP-binding protein RhoE",
  "term_id": "GO:0005886"
}